{
  "gene_symbol": "PLA2G2D",
  "gene": "UniProtKB:Q9UNK4",
  "term_label": "Unknown cellular component",
  "gene_name": "Group IID secretory phospholipase A2",
  "term_id": "UNKNOWN:0003"
}